regulation of miRNA processing [GO:1903798] (biological process) Also known as: regulation of microRNA processing, regulation of gene silencing by miRNA, production of miRNAs, regulation of microRNA-mediated gene silencing, production of microRNAs, regulation of miRNA maturation, regulation of miRNA biogenesis, regulation of microRNA biogenesis, regulation of microRNA biosynthesis, regulation of microRNA biosynthetic process, regulation of microRNA metabolic process, regulation of microRNA metabolism Definition: Any process that modulates the frequency, rate or extent of microRNA processing. References: PMID:22269326 Sources: GOC:BHF, GOC:BHF_miRNA, GOC:TermGenie, GOC:rph, GO_REF:0000058 Subtypes: negative regulation of miRNA processing [GO:1903799], positive regulation of miRNA processing [GO:1903800], regulation of pre-miRNA processing [GO:2000631], regulation of primary miRNA processing [GO:2000634] Relationships: is a type of regulation of regulatory ncRNA processing [GO:0070920]; regulates miRNA processing [GO:0035196]